{
  "term_id": "GO:0070585",
  "gene_name": "DnaJ homolog subfamily A member 1",
  "gene_symbol": "DNAJA1",
  "term_label": "protein localization to mitochondrion",
  "gene": "UniProtKB:P31689"
}